{
  "term_label": "caveola",
  "gene": "UniProtKB:Q14114",
  "gene_symbol": "LRP8",
  "term_id": "GO:0005901",
  "gene_name": "Low-density lipoprotein receptor-related protein 8"
}